{
  "gene": "UniProtKB:Q9ULN7",
  "term_label": "Unknown biological process",
  "gene_symbol": "PNMA8B",
  "gene_name": "Paraneoplastic antigen-like protein 8B",
  "term_id": "UNKNOWN:0002"
}